{
  "gene_name": "Diacylglycerol kinase iota",
  "term_label": "diacylglycerol metabolic process",
  "gene": "UniProtKB:O75912",
  "gene_symbol": "DGKI",
  "term_id": "GO:0046339"
}